{
  "gene": "UniProtKB:Q9NYF5",
  "gene_symbol": "FAM13B",
  "gene_name": "Protein FAM13B",
  "term_id": "UNKNOWN:0003",
  "term_label": "Unknown cellular component"
}